{
  "gene_symbol": "LRRC52",
  "gene_name": "Leucine-rich repeat-containing protein 52",
  "term_id": "GO:0044325",
  "term_label": "transmembrane transporter binding",
  "gene": "UniProtKB:Q8N7C0"
}